induction of positive chemotaxis [GO:0050930] (biological process) Sources: GOC:ai Relationships: is a type of positive regulation of positive chemotaxis [GO:0050927] Definition: Any process that initiates the directed movement of a motile cell or organism towards a higher concentration in a concentration gradient of a specific chemical.